{
  "gene_symbol": "TAF11L14",
  "gene_name": "TATA-box-binding protein-associated factor 11-like protein 14",
  "term_id": "GO:0005669",
  "term_label": "transcription factor TFIID complex",
  "gene": "UniProtKB:A0A1W2PPL8"
}